{
  "term_label": "autophagosome assembly",
  "gene": "UniProtKB:A1A4Y4",
  "gene_name": "Immunity-related GTPase family M protein",
  "term_id": "GO:0000045",
  "gene_symbol": "IRGM"
}